{
  "term_label": "Unknown molecular function",
  "term_id": "UNKNOWN:0001",
  "gene_name": "Zinc finger SWIM domain-containing protein 7",
  "gene": "UniProtKB:Q19AV6",
  "gene_symbol": "ZSWIM7"
}